nuclear RNA-directed RNA polymerase complex [GO:0031380] (cellular component) Relationships: is a type of RNA-directed RNA polymerase complex [GO:0031379]; is_a nuclear protein-containing complex [GO:0140513] Definition: A complex required for RNAi mediated heterochromatin assembly. In S. pombe this contains RNA-directed RNA polymerase, a putative helicase and a protein containing a pap25 associated domain. Also known as: RDRC, Rdr1 complex References: PMID:15607976 Sources: GOC:vw